{
  "gene": "UniProtKB:P49736",
  "gene_name": "DNA replication licensing factor MCM2",
  "gene_symbol": "MCM2",
  "term_label": "single-stranded DNA helicase activity",
  "term_id": "GO:0017116"
}